{
  "term_id": "UNKNOWN:0002",
  "gene_name": "Annexin A13",
  "gene": "UniProtKB:P27216",
  "gene_symbol": "ANXA13",
  "term_label": "Unknown biological process"
}